non-ribosomal peptide synthetase activity [GO:1904091] (molecular function) Note: Examples are the ferrichrome synthetase Sib1 in S. pombe and the peptidyl carrier protein (PCP) module in bacterial nonribosomal peptide synthases (NRPSs), which holds the peptidyl group and acts as a swinging arm, limiting diffusion until the peptide comes into contact with the next enzymatic module in the NRPS process. Relationships: is a type of catalytic activity [GO:0003824]; is part of nonribosomal peptide biosynthetic process [GO:0019184] Definition: Catalysis of a multistep reaction that produce non-ribosomal peptides. The key chain-building reaction, a C-N bond-forming reaction, involves the generation of the characteristic peptide bond by nucleophilic attack of the amino group of an amino-acyl donor unit covalently bound to a downstream peptidyl carrier protein module (amino acyl-S-PCP) on the acyl group of an upstream electrophilic acyl- or peptidyl acyl-S-PCP chain, catalyzed by a condensation (C) domain. Supplementing these core chain-elongation domains are variable numbers of auxiliary domains that are responsible for modification of the growing polypeptide chain by a small set of iterated reactions including epimerization, N-methylation, and heterocyclization. Also known as: peptidyl carrier protein activity involved in nonribosomal peptide biosynthesis, peptidyl carrier protein activity involved in nonribosomal peptide biosynthetic process, PCP, peptidyl carrier protein, peptidyl carrier protein activity Subtypes: glutathione synthase activity [GO:0004363], amino acid ligation activity by nonribosomal peptide synthase [GO:0097429] References: PMID:10631508, PMID:17502372